{
  "gene": "UniProtKB:P05198",
  "gene_symbol": "EIF2S1",
  "term_id": "GO:0033290",
  "gene_name": "Eukaryotic translation initiation factor 2 subunit 1",
  "term_label": "eukaryotic 48S preinitiation complex"
}